{
  "gene": "UniProtKB:Q8IWV2",
  "term_id": "GO:0045202",
  "gene_symbol": "CNTN4",
  "gene_name": "Contactin-4",
  "term_label": "synapse"
}